{
  "gene_name": "Charged multivesicular body protein 7",
  "gene": "UniProtKB:Q8WUX9",
  "term_label": "ESCRT III complex",
  "term_id": "GO:0000815",
  "gene_symbol": "CHMP7"
}